{
  "gene_symbol": "KIF12",
  "term_label": "microtubule binding",
  "term_id": "GO:0008017",
  "gene": "UniProtKB:Q96FN5",
  "gene_name": "Kinesin-like protein KIF12"
}